{
  "gene_name": "Myb_SANT-like DNA-binding domain-containing protein 1",
  "gene_symbol": "MSANTD1",
  "term_label": "nuclear body",
  "gene": "UniProtKB:Q6ZTZ1",
  "term_id": "GO:0016604"
}